peroxisome proliferator activated receptor signaling pathway [GO:0035357] (BP) Definition: A nuclear receptor-mediated signaling pathway initiated by a ligand binding to an intracellular peroxisome proliferator activated receptor (alpha, beta or gamma) of the nuclear receptor protein family, and ending with regulation of a downstream cellular process, e.g. transcription. References: PMID:18221086 Relationships: is_a GO:0141193 Regulation: regulated by GO:0035358; negatively regulated by negative regulation of peroxisome proliferator activated receptor signaling pathway [GO:0035359]; positively regulated by GO:0035360 Also known as: PPAR signaling pathway, peroxisome proliferator activated receptor signalling pathway, peroxisome proliferator-activated receptor signaling pathway